{
  "gene_name": "Phospholipid-transporting ATPase IH",
  "gene_symbol": "ATP11A",
  "gene": "UniProtKB:P98196",
  "term_label": "phospholipid translocation",
  "term_id": "GO:0045332"
}